(1->6)-beta-D-glucan metabolic process [GO:0006077] (biological process) Definition: The chemical reactions and pathways involving (1->6)-beta-D-glucans, compounds composed of glucose residues linked by (1->6)-beta-D-glucosidic bonds. Sources: ISBN:0198506732 Also known as: 1,6-beta-glucan metabolic process, 1,6-beta-glucan metabolism, beta-1,6 glucan metabolic process, beta-1,6 glucan metabolism Relationships: is a type of beta-glucan metabolic process [GO:0051273] Subtypes: (1->6)-beta-D-glucan biosynthetic process [GO:0006078], GO:0006079